{
  "term_id": "GO:0051321",
  "gene_name": "Synaptonemal complex protein 3",
  "gene_symbol": "SYCP3",
  "gene": "UniProtKB:Q8IZU3",
  "term_label": "meiotic cell cycle"
}